{
  "gene_name": "Embryonal Fyn-associated substrate",
  "gene": "UniProtKB:O43281",
  "term_label": "plasma membrane",
  "gene_symbol": "EFS",
  "term_id": "GO:0005886"
}